{
  "gene_symbol": "PHACTR2",
  "term_id": "UNKNOWN:0003",
  "gene_name": "Phosphatase and actin regulator 2",
  "gene": "UniProtKB:O75167",
  "term_label": "Unknown cellular component"
}